{
  "term_label": "PML body",
  "term_id": "GO:0016605",
  "gene_symbol": "LRCH4",
  "gene_name": "Leucine-rich repeat and calponin homology domain-containing protein 4",
  "gene": "UniProtKB:O75427"
}